myeloid dendritic cell activation [GO:0001773] (biological process) Sources: GOC:mgi_curators, ISBN:0781735149 Definition: The change in morphology and behavior of a dendritic cell resulting from exposure to a cytokine, chemokine, cellular ligand, or soluble factor. Relationships: is a type of myeloid leukocyte activation [GO:0002274] Regulation: regulated by GO:0030885; negatively regulated by negative regulation of myeloid dendritic cell activation [GO:0030886]; RO_0002213 by positive regulation of myeloid dendritic cell activation [GO:0030887] Subtypes: myeloid dendritic cell activation involved in immune response [GO:0002277], myeloid dendritic cell differentiation [GO:0043011]